{
  "gene_symbol": "S100A9",
  "term_id": "GO:0043542",
  "gene": "UniProtKB:P06702",
  "term_label": "endothelial cell migration",
  "gene_name": "Protein S100-A9"
}